{
  "term_label": "endocytosis",
  "term_id": "GO:0006897",
  "gene": "UniProtKB:Q7L0Q8",
  "gene_name": "Rho-related GTP-binding protein RhoU",
  "gene_symbol": "RHOU"
}